{
  "gene_symbol": "DOCK4",
  "term_label": "small GTPase binding",
  "term_id": "GO:0031267",
  "gene_name": "Dedicator of cytokinesis protein 4",
  "gene": "UniProtKB:Q8N1I0"
}